flight [GO:0060361] (biological process) Subtypes: flight involved in flight behavior [GO:0060362] Sources: GOC:dph Definition: Self-propelled movement of an organism from one location to another through the air, usually by means of active wing movement. Relationships: is a type of locomotion [GO:0040011]